{
  "gene": "UniProtKB:Q5T686",
  "term_label": "positive regulation of MAPK cascade",
  "term_id": "GO:0043410",
  "gene_name": "Arginine vasopressin-induced protein 1",
  "gene_symbol": "AVPI1"
}